{
  "gene_name": "Beta-arrestin-1",
  "term_id": "GO:0002031",
  "term_label": "G protein-coupled receptor internalization",
  "gene": "UniProtKB:P49407",
  "gene_symbol": "ARRB1"
}